{
  "gene_name": "Putative uncharacterized protein ANP32CP",
  "term_id": "GO:0006913",
  "term_label": "nucleocytoplasmic transport",
  "gene": "UniProtKB:O43423",
  "gene_symbol": "ANP32CP"
}